{
  "gene_name": "Xylosyl- and glucuronyltransferase LARGE1",
  "gene_symbol": "LARGE1",
  "term_label": "xylosyltransferase activity",
  "term_id": "GO:0042285",
  "gene": "UniProtKB:O95461"
}